{
  "gene": "UniProtKB:Q2M3T9",
  "gene_name": "Hyaluronidase-4",
  "gene_symbol": "HYAL4",
  "term_label": "hyaluronan catabolic process",
  "term_id": "GO:0030214"
}